{
  "gene": "UniProtKB:Q9ULK6",
  "gene_symbol": "RNF150",
  "term_id": "GO:0006511",
  "gene_name": "RING finger protein 150",
  "term_label": "ubiquitin-dependent protein catabolic process"
}